{
  "gene_symbol": "ARHGAP18",
  "term_id": "GO:0005096",
  "gene_name": "Rho GTPase-activating protein 18",
  "gene": "UniProtKB:Q8N392",
  "term_label": "GTPase activator activity"
}